{
  "gene_symbol": "STKLD1",
  "term_label": "Unknown biological process",
  "gene_name": "Serine_threonine kinase-like domain-containing protein STKLD1",
  "gene": "UniProtKB:Q8NE28",
  "term_id": "UNKNOWN:0002"
}